{
  "term_id": "GO:0030335",
  "gene_name": "Semaphorin-6B",
  "gene_symbol": "SEMA6B",
  "term_label": "positive regulation of cell migration",
  "gene": "UniProtKB:Q9H3T3"
}